{
  "term_id": "GO:0007411",
  "gene": "UniProtKB:Q15768",
  "term_label": "axon guidance",
  "gene_symbol": "EFNB3",
  "gene_name": "Ephrin-B3"
}